{
  "gene": "UniProtKB:Q13557",
  "term_id": "GO:0005737",
  "gene_symbol": "CAMK2D",
  "gene_name": "Calcium_calmodulin-dependent protein kinase type II subunit delta",
  "term_label": "cytoplasm"
}